filiform apparatus [GO:0043680] (cellular component) Sources: ISBN:0471245208 Relationships: is a type of cellular anatomical structure [GO:0110165]; is part of cell wall [GO:0005618] Definition: A complex of cell wall invaginations in a synergid cell, similar to those in transfer cells.